RNA ligase (ATP) activity [GO:0003972] (molecular function) Definition: Catalysis of the reaction: ATP + (ribonucleotide)n-3'-hydroxyl + 5'-phospho-(ribonucleotide)m = (ribonucleotide)n+m + AMP + diphosphate. Sources: EC:6.5.1.3 Relationships: is a type of RNA ligase activity [GO:0008452] Also known as: ribonucleic ligase activity, poly(ribonucleotide):poly(ribonucleotide) ligase (AMP-forming), polyribonucleotide ligase activity, polyribonucleotide synthase (ATP) activity